L-homocysteine biosynthetic process [GO:0071269] (biological process) Also known as: L-homocysteine anabolism, L-homocysteine biosynthesis, L-homocysteine formation, L-homocysteine synthesis Sources: GOC:ecd, GOC:mah Relationships: is a type of serine family amino acid biosynthetic process [GO:0009070]; is a type of GO:0071268; is a type of L-amino acid biosynthetic process [GO:0170034] Definition: The chemical reactions and pathways resulting in the formation of L-homocysteine, the L-enantiomer of 2-amino-4-sulfanylbutanoic acid.